{
  "term_label": "cytoplasm",
  "gene_name": "IQ and AAA domain-containing protein 1-like",
  "term_id": "GO:0005737",
  "gene_symbol": "IQCA1L",
  "gene": "UniProtKB:A6NCM1"
}